{
  "term_label": "reciprocal meiotic recombination",
  "gene_symbol": "MND1",
  "gene_name": "Meiotic nuclear division protein 1 homolog",
  "gene": "UniProtKB:Q9BWT6",
  "term_id": "GO:0007131"
}